receptor antagonist activity [GO:0048019] (molecular function) Sources: GOC:ceb, ISBN:0198506732 Subtypes: interleukin-1 receptor antagonist activity [GO:0005152], fibroblast growth factor receptor antagonist activity [GO:0030353], activin receptor antagonist activity [GO:0038102], GO:0046817 Definition: The activity of a gene product that interacts with a receptor to decrease the ability of the receptor agonist to bind and activate the receptor. Relationships: is a type of signaling receptor binding [GO:0005102]; is a type of signaling receptor inhibitor activity [GO:0030547] Also known as: receptor ligand activity